{
  "gene_name": "Titin",
  "term_id": "GO:0045214",
  "term_label": "sarcomere organization",
  "gene": "UniProtKB:Q8WZ42",
  "gene_symbol": "TTN"
}